{
  "term_id": "UNKNOWN:0002",
  "gene_name": "Complement C1s subcomponent",
  "gene": "UniProtKB:P09871",
  "term_label": "Unknown biological process",
  "gene_symbol": "C1S"
}